{
  "gene_name": "Olfactomedin-like protein 3",
  "term_id": "GO:0007165",
  "gene": "UniProtKB:Q9NRN5",
  "gene_symbol": "OLFML3",
  "term_label": "signal transduction"
}